meiotic strand invasion involved in meiotic gene conversion [GO:0010775] (biological process) Definition: The cell cycle process in which double strand breaks are formed and repaired through a double Holliday junction intermediate resulting in meiotic recombination. Sources: GOC:dph, GOC:tb Relationships: is a type of meiotic strand invasion [GO:0000708]; is part of meiotic gene conversion [GO:0006311]